{
  "gene_symbol": "CNGA3",
  "term_label": "intracellularly cAMP-activated cation channel activity",
  "term_id": "GO:0005222",
  "gene_name": "Cyclic nucleotide-gated cation channel alpha-3",
  "gene": "UniProtKB:Q16281"
}